{
  "gene_name": "Zinc finger protein 793",
  "term_id": "GO:0000978",
  "term_label": "RNA polymerase II cis-regulatory region sequence-specific DNA binding",
  "gene_symbol": "ZNF793",
  "gene": "UniProtKB:Q6ZN11"
}